{
  "gene_name": "Serine_threonine-protein kinase LMTK2",
  "term_id": "UNKNOWN:0003",
  "gene_symbol": "LMTK2",
  "term_label": "Unknown cellular component",
  "gene": "UniProtKB:Q8IWU2"
}